{
  "gene_name": "Uncharacterized protein KIAA0825",
  "term_label": "Unknown biological process",
  "term_id": "UNKNOWN:0002",
  "gene": "UniProtKB:Q8IV33",
  "gene_symbol": "KIAA0825"
}